{
  "gene": "UniProtKB:Q8TCA0",
  "gene_symbol": "LRRC20",
  "term_id": "UNKNOWN:0003",
  "gene_name": "Leucine-rich repeat-containing protein 20",
  "term_label": "Unknown cellular component"
}